{
  "gene_name": "Protein MIS12 homolog",
  "term_id": "GO:0000444",
  "gene_symbol": "MIS12",
  "gene": "UniProtKB:Q9H081",
  "term_label": "MIS12/MIND type complex"
}